{
  "gene_symbol": "CDK9",
  "term_id": "GO:0004693",
  "gene_name": "Cyclin-dependent kinase 9",
  "gene": "UniProtKB:P50750",
  "term_label": "cyclin-dependent protein serine/threonine kinase activity"
}